{
  "gene_name": "Nuclear cap-binding protein subunit 1",
  "gene": "UniProtKB:Q09161",
  "term_label": "mRNA binding",
  "gene_symbol": "NCBP1",
  "term_id": "GO:0003729"
}